{
  "gene": "UniProtKB:Q13324",
  "gene_symbol": "CRHR2",
  "term_id": "GO:0060291",
  "gene_name": "Corticotropin-releasing factor receptor 2",
  "term_label": "long-term synaptic potentiation"
}